DNA-binding transcription activator activity, RNA polymerase II-specific [GO:0001228] (molecular function) Note: For usage guidance, see comment in GO:0003700 ; DNA-binding transcription factor activity. Also known as: RNA polymerase II transcription regulatory region sequence-specific DNA binding transcription factor activity involved in positive regulation of transcription, transcriptional activator activity, RNA polymerase II transcription regulatory region sequence-specific DNA binding, RNA polymerase II core promoter proximal region sequence-specific DNA binding transcription factor activity involved in positive regulation of transcription, RNA polymerase II distal enhancer sequence-specific DNA-binding transcription factor activity involved in positive regulation of transcription, RNA polymerase II transcriptional activator activity, copper ion regulated proximal promoter sequence-specific DNA binding, RNA polymerase II transcriptional activator activity, metal ion regulated core promoter proximal region sequence-specific binding, RNA polymerase II transcriptional activator activity, metal ion regulated proximal promoter sequence-specific DNA binding, RNA polymerase II transcriptional activator activity, zinc ion regulated core promoter proximal region sequence-specific binding, RNA polymerase II transcriptional activator activity, zinc ion regulated proximal promoter sequence-specific DNA binding, copper ion regulated core promoter proximal region sequence-specific DNA binding RNA polymerase II transcription factor activity involved in positive regulation of transcription, distal enhancer DNA-binding transcription activator activity, RNA polymerase II-specific, metal ion regulated core promoter proximal region sequence-specific DNA binding RNA polymerase II transcription factor activity involved in positive regulation of transcription, metal ion regulated sequence-specific DNA binding transcription factor activity involved in positive regulation of transcription, proximal promoter DNA-binding transcription activator activity, RNA polymerase II-specific, sequence-specific distal enhancer binding RNA polymerase II transcription factor activity involved in positive regulation of transcription, transcriptional activator activity, RNA polymerase II core promoter proximal region sequence-specific binding, transcriptional activator activity, RNA polymerase II distal enhancer sequence-specific DNA binding, transcriptional activator activity, RNA polymerase II proximal promoter sequence-specific DNA binding, transcriptional activator activity, metal ion regulated sequence-specific DNA binding, zinc ion regulated core promoter proximal region sequence-specific DNA binding RNA polymerase II transcription factor activity involved in positive regulation of transcription Definition: A DNA-binding transcription factor activity that activates or increases transcription of specific gene sets transcribed by RNA polymerase II. Relationships: is a type of DNA-binding transcription factor activity, RNA polymerase II-specific [GO:0000981]; is a type of GO:0001216; is part of GO:0045944 References: PMID:20737563, PMID:27145859 Sources: GOC:aruk, GOC:txnOH-2018